{
  "gene_symbol": "GTF2A2",
  "term_label": "transcription factor TFIIA complex",
  "gene": "UniProtKB:P52657",
  "gene_name": "Transcription initiation factor IIA subunit 2",
  "term_id": "GO:0005672"
}